{
  "gene": "UniProtKB:Q6ZW49",
  "term_id": "UNKNOWN:0001",
  "gene_symbol": "PAXIP1",
  "gene_name": "PAX-interacting protein 1",
  "term_label": "Unknown molecular function"
}